{
  "gene_name": "High affinity copper uptake protein 1",
  "gene_symbol": "SLC31A1",
  "term_label": "copper ion transmembrane transport",
  "gene": "UniProtKB:O15431",
  "term_id": "GO:0035434"
}